{
  "gene": "UniProtKB:Q6L8H4",
  "term_label": "Unknown molecular function",
  "term_id": "UNKNOWN:0001",
  "gene_name": "Keratin-associated protein 5-1",
  "gene_symbol": "KRTAP5-1"
}